{
  "term_label": "adenylate cyclase-inhibiting G protein-coupled receptor signaling pathway",
  "term_id": "GO:0007193",
  "gene_symbol": "CORT",
  "gene_name": "Cortistatin",
  "gene": "UniProtKB:O00230"
}